{
  "gene_symbol": "FIBCD1",
  "gene": "UniProtKB:Q8N539",
  "gene_name": "Fibrinogen C domain-containing protein 1",
  "term_id": "UNKNOWN:0001",
  "term_label": "Unknown molecular function"
}